amino acid salvage [GO:0043102] (biological process) Definition: Any process which produces an amino acid from derivatives of it, without de novo synthesis. Sources: GOC:jl Relationships: is a type of amino acid biosynthetic process [GO:0008652]; is a type of metabolic compound salvage [GO:0043094] Subtypes: proline salvage [GO:0019492], GO:0071267